{
  "term_id": "GO:0005615",
  "gene_symbol": "FSHB",
  "term_label": "extracellular space",
  "gene": "UniProtKB:P01225",
  "gene_name": "Follitropin subunit beta"
}